positive regulation of capsule organization [GO:1901915] (biological process) Relationships: is a type of positive regulation of cellular component organization [GO:0051130]; is a type of regulation of capsule organization [GO:1901913]; positively regulates capsule organization [GO:0045230] Sources: GOC:TermGenie, GOC:di Also known as: positive regulation of capsule organisation, up regulation of capsule organisation, up regulation of capsule organization, up-regulation of capsule organisation, up-regulation of capsule organization, upregulation of capsule organisation, upregulation of capsule organization, activation of capsule organisation, activation of capsule organization, activation of capsule organization and biogenesis, positive regulation of capsule organization and biogenesis, up regulation of capsule organization and biogenesis, up-regulation of capsule organization and biogenesis, upregulation of capsule organization and biogenesis Subtypes: positive regulation of capsule polysaccharide biosynthetic process [GO:0062085] Definition: Any process that activates or increases the frequency, rate or extent of capsule organization.